{
  "gene_name": "Dehydrogenase_reductase SDR family member 7B",
  "gene_symbol": "DHRS7B",
  "term_label": "membrane",
  "gene": "UniProtKB:Q6IAN0",
  "term_id": "GO:0016020"
}